{
  "term_label": "intracellular protein localization",
  "gene": "UniProtKB:Q86XA9",
  "term_id": "GO:0008104",
  "gene_name": "HEAT repeat-containing protein 5A",
  "gene_symbol": "HEATR5A"
}